{
  "term_label": "brain morphogenesis",
  "gene_name": "Platelet-activating factor acetylhydrolase IB subunit beta",
  "gene_symbol": "PAFAH1B1",
  "term_id": "GO:0048854",
  "gene": "UniProtKB:P43034"
}